all-trans-retinol binding [GO:1904768] (molecular function) References: PMID:19828452 Sources: GOC:TermGenie, GOC:kmv, GO_REF:0000067 Definition: Binding to all-trans-retinol. Relationships: is a type of retinol binding [GO:0019841]